{
  "gene_symbol": "CDK2",
  "gene": "UniProtKB:P24941",
  "gene_name": "Cyclin-dependent kinase 2",
  "term_label": "cyclin-dependent protein serine/threonine kinase activity",
  "term_id": "GO:0004693"
}